cytosolic proteasome complex [GO:0031597] (cellular component) Relationships: is a type of GO:0000502; is part of GO:0005829 Sources: GOC:mah, GOC:mtg_sensu Subtypes: GO:0009376 Definition: A proteasome complex found in the cytosol of a cell.